{
  "term_id": "GO:0004843",
  "gene": "UniProtKB:Q96G74",
  "gene_name": "OTU domain-containing protein 5",
  "gene_symbol": "OTUD5",
  "term_label": "cysteine-type deubiquitinase activity"
}